{
  "term_id": "GO:0038023",
  "term_label": "signaling receptor activity",
  "gene_name": "Platelet glycoprotein Ib alpha chain",
  "gene_symbol": "GP1BA",
  "gene": "UniProtKB:P07359"
}